{
  "gene_symbol": "APOBEC3C",
  "term_label": "cytidine deaminase activity",
  "gene": "UniProtKB:Q9NRW3",
  "term_id": "GO:0004126",
  "gene_name": "DNA dC-dU-editing enzyme APOBEC-3C"
}